{
  "term_label": "regulation of synaptic transmission, glutamatergic",
  "gene_symbol": "HOMER1",
  "term_id": "GO:0051966",
  "gene_name": "Homer protein homolog 1",
  "gene": "UniProtKB:Q86YM7"
}